specification of metanephric proximal tubule identity [GO:0072297] (biological process) Sources: GOC:bf, GOC:mtg_kidney_jan10 Relationships: is a type of specification of proximal tubule identity [GO:0072082]; is_a GO:0072293; is part of metanephric proximal tubule morphogenesis [GO:0072288] Definition: The process in which the proximal tubule of the metanephric nephron acquires its identity.